{
  "gene": "UniProtKB:Q9NP95",
  "gene_name": "Fibroblast growth factor 20",
  "gene_symbol": "FGF20",
  "term_label": "fibroblast growth factor receptor binding",
  "term_id": "GO:0005104"
}